Toll-like receptor 2 binding [GO:0035663] (molecular function) Definition: Binding to a Toll-like 2 protein, a pattern recognition receptor that binds microbial pattern motifs to initiate an innate immune response. Also known as: TLR2 binding Sources: GOC:BHF Relationships: is a type of GO:0035325